{
  "term_label": "Unknown molecular function",
  "term_id": "UNKNOWN:0001",
  "gene_name": "Uncharacterized protein",
  "gene": "UniProtKB:A0A6Q8PGZ7",
  "gene_symbol": "A0A6Q8PGZ7"
}